{
  "gene": "UniProtKB:O00175",
  "gene_symbol": "CCL24",
  "term_id": "GO:0030335",
  "gene_name": "C-C motif chemokine 24",
  "term_label": "positive regulation of cell migration"
}